{
  "term_id": "UNKNOWN:0003",
  "gene": "UniProtKB:Q9Y228",
  "gene_name": "TRAF3-interacting JNK-activating modulator",
  "term_label": "Unknown cellular component",
  "gene_symbol": "TRAF3IP3"
}